{
  "term_id": "GO:0045098",
  "term_label": "type III intermediate filament",
  "gene": "UniProtKB:P41219",
  "gene_name": "Peripherin",
  "gene_symbol": "PRPH"
}